negative regulation of morphogenesis of an epithelium [GO:1905331] (biological process) Also known as: down regulation of epithelium morphogenesis, down regulation of morphogenesis of an epithelium, down-regulation of epithelium morphogenesis, down-regulation of morphogenesis of an epithelium, downregulation of epithelium morphogenesis, downregulation of morphogenesis of an epithelium, negative regulation of epithelium morphogenesis, inhibition of epithelium morphogenesis, inhibition of morphogenesis of an epithelium References: PMID:25745997 Sources: GOC:TermGenie, GOC:bhm, GO_REF:0000058 Definition: Any process that stops, prevents or reduces the frequency, rate or extent of morphogenesis of an epithelium. Relationships: is a type of negative regulation of developmental process [GO:0051093]; is a type of regulation of morphogenesis of an epithelium [GO:1905330]; negatively regulates morphogenesis of an epithelium [GO:0002009] Subtypes: GO:0060686, GO:0061048, negative regulation of branching involved in ureteric bud morphogenesis [GO:0090191], negative regulation of heart looping [GO:1901208], negative regulation of convergent extension involved in axis elongation [GO:1901233], negative regulation of epiboly involved in gastrulation with mouth forming second [GO:1904087], negative regulation of convergent extension involved in gastrulation [GO:1904104], negative regulation of otic vesicle morphogenesis [GO:1904119], GO:1905277, negative regulation of blood vessel branching [GO:1905554], negative regulation of endothelial tube morphogenesis [GO:1905955] Note: An example of this is MMRN2 in human (Q9H8L6) in PMID:25745997 (inferred from direct assay).